{
  "term_label": "endocytic recycling",
  "gene": "UniProtKB:Q7Z3J2",
  "gene_name": "VPS35 endosomal protein-sorting factor-like",
  "gene_symbol": "VPS35L",
  "term_id": "GO:0032456"
}